cell proliferation involved in compound eye morphogenesis [GO:0035736] (biological process) Definition: The multiplication or reproduction of cells, resulting in the expansion of a cell population that contributes to compound eye morphogenesis. Sources: GOC:bf, GOC:sart Relationships: is a type of cell population proliferation [GO:0008283]; is part of compound eye morphogenesis [GO:0001745] Regulation: regulated by regulation of cell proliferation involved in compound eye morphogenesis [GO:2000495]; negatively regulated by negative regulation of cell proliferation involved in compound eye morphogenesis [GO:2000496]; positively regulated by positive regulation of cell proliferation involved in compound eye morphogenesis [GO:2000497]